{
  "gene_name": "Tripartite motif-containing protein 3",
  "gene_symbol": "TRIM3",
  "gene": "UniProtKB:O75382",
  "term_label": "proteasome-mediated ubiquitin-dependent protein catabolic process",
  "term_id": "GO:0043161"
}